{
  "gene_name": "Guanine nucleotide exchange factor VAV3",
  "term_id": "GO:0051897",
  "gene": "UniProtKB:Q9UKW4",
  "term_label": "positive regulation of phosphatidylinositol 3-kinase/protein kinase B signal transduction",
  "gene_symbol": "VAV3"
}